{
  "term_label": "Unknown biological process",
  "gene_name": "Putative uncharacterized protein encoded by LINC00528",
  "gene": "UniProtKB:Q8N1L1",
  "gene_symbol": "LINC00528",
  "term_id": "UNKNOWN:0002"
}